{
  "term_id": "GO:0043123",
  "term_label": "positive regulation of canonical NF-kappaB signal transduction",
  "gene_symbol": "TRIM5",
  "gene_name": "Tripartite motif-containing protein 5",
  "gene": "UniProtKB:Q9C035"
}